{
  "term_label": "ISG15 transferase activity",
  "gene": "UniProtKB:Q96LR5",
  "term_id": "GO:0042296",
  "gene_symbol": "UBE2E2",
  "gene_name": "Ubiquitin-conjugating enzyme E2 E2"
}